{
  "term_label": "chromatin",
  "term_id": "GO:0000785",
  "gene_symbol": "VRTN",
  "gene": "UniProtKB:Q9H8Y1",
  "gene_name": "Vertnin"
}